positive regulation of phospholipid transport [GO:2001140] (biological process) Subtypes: positive regulation of phospholipid translocation [GO:0061092], GO:1902995 Definition: Any process that activates or increases the frequency, rate or extent of phospholipid transport. Sources: GOC:obol Relationships: is a type of GO:0032370; is a type of regulation of phospholipid transport [GO:2001138]; positively regulates phospholipid transport [GO:0015914]